{
  "term_id": "GO:0035556",
  "gene": "UniProtKB:Q6ZNQ3",
  "gene_name": "Leucine-rich repeat-containing protein 69",
  "term_label": "intracellular signal transduction",
  "gene_symbol": "LRRC69"
}